{
  "gene_symbol": "ATP9B",
  "term_label": "retrograde vesicle-mediated transport, Golgi to endoplasmic reticulum",
  "gene_name": "Probable phospholipid-transporting ATPase IIB",
  "gene": "UniProtKB:O43861",
  "term_id": "GO:0006890"
}